negative regulation of monocyte aggregation [GO:1900624] (biological process) Also known as: down regulation of monocyte aggregation, down regulation of mononuclear phagocyte aggregation, down-regulation of monocyte aggregation, down-regulation of mononuclear phagocyte aggregation, downregulation of monocyte aggregation, downregulation of mononuclear phagocyte aggregation, inhibition of mononuclear phagocyte aggregation, negative regulation of mononuclear phagocyte aggregation, inhibition of monocyte aggregation Definition: Any process that stops, prevents or reduces the frequency, rate or extent of monocyte aggregation. Sources: GOC:BHF, GOC:TermGenie Relationships: is a type of regulation of monocyte aggregation [GO:1900623]; is a type of negative regulation of leukocyte cell-cell adhesion [GO:1903038]; negatively regulates monocyte aggregation [GO:0070487]